{
  "term_id": "UNKNOWN:0003",
  "gene": "UniProtKB:P60509",
  "gene_symbol": "ERVPABLB-1",
  "gene_name": "Endogenous retrovirus group PABLB member 1 Env polyprotein",
  "term_label": "Unknown cellular component"
}